right posteriolateral flagellum [GO:0097557] (cellular component) Relationships: is a type of 9+2 motile cilium [GO:0097729] References: PMID:16607022, PMID:5961344 Sources: GOC:giardia, ISBN:9780124260207 Also known as: right posteriolateral cilium, right posterolateral cilium, right posterolateral flagellum Note: Note that we deem cilium and microtubule-based flagellum to be equivalent; the primary term name reflects frequency of use. Also note that, due to the asymmetric nature of the Giardia trophozoite, this term is defined spatially as the trophozoite is viewed from the dorsal side, with the two nuclei dorsal to the ventral disc, and the ventral disc toward the anterior. Definition: A cilium (also called flagellum) found in Giardia species (trophozoite stage). It is nucleated by the right posteriolateral basal body and extends cytoplasmically toward the cell posterior, marking the right anterior boundary of the lateral shield and the right lateral region of the funis before exiting at the right lateral region of the cell body.